{
  "gene_name": "Mpv17-like protein 2",
  "term_label": "mitochondrion",
  "gene_symbol": "MPV17L2",
  "term_id": "GO:0005739",
  "gene": "UniProtKB:Q567V2"
}